{
  "term_id": "GO:0005856",
  "gene_symbol": "ITGB1BP1",
  "term_label": "cytoskeleton",
  "gene_name": "Integrin beta-1-binding protein 1",
  "gene": "UniProtKB:O14713"
}